{
  "gene_symbol": "SYNE3",
  "term_label": "nuclear outer membrane",
  "gene_name": "Nesprin-3",
  "term_id": "GO:0005640",
  "gene": "UniProtKB:Q6ZMZ3"
}